{
  "gene_name": "Deoxynucleotidyltransferase terminal-interacting protein 1",
  "term_id": "UNKNOWN:0002",
  "term_label": "Unknown biological process",
  "gene_symbol": "DNTTIP1",
  "gene": "UniProtKB:Q9H147"
}